brassinosteroid homeostasis [GO:0010268] (BP) Definition: Any process involved in the maintenance of an internal steady state of brassinosteroids within an organism or cell. Relationships: is a type of lipid homeostasis [GO:0055088] References: PMID:15908602